response to L-glutamine [GO:1904844] (BP) Definition: Any process that results in a change in state or activity of a cell or an organism (in terms of movement, secretion, enzyme production, gene expression, etc.) as a result of a L-glutamine stimulus. Relationships: is a type of GO:0043200; is a type of response to nitrogen compound [GO:1901698]; is a type of response to oxygen-containing compound [GO:1901700] Subtypes: GO:1904845 References: PMID:23185570 Sources: GOC:TermGenie, GO_REF:0000071